{
  "gene": "UniProtKB:O75884",
  "gene_symbol": "RBBP9",
  "term_id": "UNKNOWN:0002",
  "term_label": "Unknown biological process",
  "gene_name": "Serine hydrolase RBBP9"
}